{
  "gene": "UniProtKB:Q53S99",
  "gene_name": "Folate transporter-like protein C2orf83",
  "term_label": "Unknown molecular function",
  "term_id": "UNKNOWN:0001",
  "gene_symbol": "C2orf83"
}